{
  "term_label": "complement activation, classical pathway",
  "term_id": "GO:0006958",
  "gene_symbol": "IGHG1",
  "gene_name": "Immunoglobulin heavy constant gamma 1",
  "gene": "UniProtKB:P01857"
}